{
  "gene_symbol": "CEP57L1",
  "term_label": "microtubule binding",
  "gene_name": "Centrosomal protein CEP57L1",
  "gene": "UniProtKB:Q8IYX8",
  "term_id": "GO:0008017"
}